positive regulation of CD4-positive, CD25-positive, alpha-beta regulatory T cell differentiation [GO:0032831] (biological process) Also known as: positive regulation of CD4-positive, CD25-positive, alpha-beta regulatory T lymphocyte differentiation, positive regulation of CD4-positive, CD25-positive, alpha-beta regulatory T-cell differentiation, positive regulation of CD4-positive, CD25-positive, alpha-beta regulatory T-lymphocyte differentiation, up regulation of CD4-positive, CD25-positive, alpha-beta regulatory T cell differentiation, up-regulation of CD4-positive, CD25-positive, alpha-beta regulatory T cell differentiation, upregulation of CD4-positive, CD25-positive, alpha-beta regulatory T cell differentiation, activation of CD4-positive, CD25-positive, alpha-beta regulatory T cell differentiation, stimulation of CD4-positive, CD25-positive, alpha-beta regulatory T cell differentiation, positive regulation of CD4-positive, CD25-positive, alpha-beta regulatory T cell development Note: Note that immunologists typically use the word 'development' to refer to cells of B or T cell lineages undergoing the process that GO describes as 'cell differentiation'. Subtypes: positive regulation of CD4-positive, CD25-positive, alpha-beta regulatory T cell differentiation involved in immune response [GO:0032834] Relationships: is a type of regulation of CD4-positive, CD25-positive, alpha-beta regulatory T cell differentiation [GO:0032829]; is a type of GO:0043372; is a type of positive regulation of regulatory T cell differentiation [GO:0045591]; positively regulates CD4-positive, CD25-positive, alpha-beta regulatory T cell differentiation [GO:0002361] Definition: Any process that activates or increases the frequency, rate or extent of differentiation of CD4-positive, CD25-positive, alpha-beta regulatory T cells. Sources: GOC:mah